{
  "gene": "UniProtKB:Q9UJ99",
  "gene_name": "Cadherin-22",
  "term_label": "calcium-dependent cell-cell adhesion",
  "term_id": "GO:0016339",
  "gene_symbol": "CDH22"
}